{
  "gene_symbol": "CHRM3",
  "term_label": "chemical synaptic transmission",
  "gene_name": "Muscarinic acetylcholine receptor M3",
  "term_id": "GO:0007268",
  "gene": "UniProtKB:P20309"
}